beta-glucan transport [GO:0015775] (biological process) Definition: The directed movement of beta-glucans into, out of or within a cell, or between cells, by means of some agent such as a transporter or pore. Beta-glucans are compounds composed of glucose residues linked by beta-glucosidic bonds. Relationships: is a type of polysaccharide transport [GO:0015774] Sources: GOC:ai